acetylcholine receptor inhibitor activity [GO:0030550] (MF) Relationships: is a type of signaling receptor inhibitor activity [GO:0030547]; is a type of GO:0030548; negatively regulates acetylcholine receptor activity [GO:0015464] Definition: Binds to and stops, prevents or reduces the activity of an acetylcholine receptor. Sources: GOC:mah